{
  "term_id": "GO:0005769",
  "term_label": "early endosome",
  "gene_name": "Low-density lipoprotein receptor",
  "gene": "UniProtKB:P01130",
  "gene_symbol": "LDLR"
}